regulation of axon diameter [GO:0031133] (biological process) Relationships: is a type of regulation of cell projection size [GO:0032536]; is a type of regulation of axonogenesis [GO:0050770] Sources: GOC:dph, GOC:mah, GOC:tb Definition: Any process that modulates the rate, direction or extent of axon growth such that the correct diameter is attained and maintained.